{
  "gene_symbol": "YWHAB",
  "term_label": "cytoplasm",
  "gene": "UniProtKB:P31946",
  "term_id": "GO:0005737",
  "gene_name": "14-3-3 protein beta_alpha"
}